{
  "gene_name": "Olfactory receptor 5AS1",
  "term_label": "odorant binding",
  "gene_symbol": "OR5AS1",
  "term_id": "GO:0005549",
  "gene": "UniProtKB:Q8N127"
}